salicylate 1-monooxygenase activity [GO:0018658] (molecular function) Sources: EC:1.14.13.1 Definition: Catalysis of the reaction: salicylate + NADH + H+ + O2 = catechol + NAD+ + H2O + CO2. Also known as: salicylate hydroxylase activity, salicylate 1-hydroxylase activity, salicylate hydroxylase (decarboxylating), salicylate monooxygenase activity, salicylate,NADH:oxygen oxidoreductase (1-hydroxylating, decarboxylating), salicylic hydroxylase activity Relationships: is a type of GO:0016709